{
  "term_id": "GO:0008137",
  "gene": "UniProtKB:O75306",
  "term_label": "NADH dehydrogenase (ubiquinone) activity",
  "gene_name": "NADH dehydrogenase [ubiquinone] iron-sulfur protein 2, mitochondrial",
  "gene_symbol": "NDUFS2"
}